{
  "gene_symbol": "SSMEM1",
  "term_id": "UNKNOWN:0002",
  "gene": "UniProtKB:Q8WWF3",
  "gene_name": "Serine-rich single-pass membrane protein 1",
  "term_label": "Unknown biological process"
}